positive regulation of CD4-positive, alpha-beta T cell proliferation [GO:2000563] (biological process) Sources: GOC:obol Definition: Any process that activates or increases the frequency, rate or extent of CD4-positive, alpha-beta T cell proliferation. Relationships: is a type of positive regulation of alpha-beta T cell proliferation [GO:0046641]; is a type of positive regulation of CD4-positive, alpha-beta T cell activation [GO:2000516]; is a type of regulation of CD4-positive, alpha-beta T cell proliferation [GO:2000561]; positively regulates CD4-positive, alpha-beta T cell proliferation [GO:0035739]